mitochondrial mRNA polyadenylation [GO:0097222] (biological process) Definition: The enzymatic addition of a sequence of 40-60 adenylyl residues at the 3' end of a eukaryotic mitochondrial mRNA primary transcript. Mitochondria contain both stabilizing and destabilizing poly(A) tails. Relationships: is a type of GO:0000963 References: PMID:18083837 Sources: GOC:ans